{
  "gene_symbol": "SPTBN1",
  "term_label": "cortical actin cytoskeleton",
  "gene_name": "Spectrin beta chain, non-erythrocytic 1",
  "term_id": "GO:0030864",
  "gene": "UniProtKB:Q01082"
}